{
  "gene_symbol": "DPY19L2P2",
  "term_label": "spermatid development",
  "gene_name": "Putative C-mannosyltransferase DPY19L2P2",
  "gene": "UniProtKB:Q6ZN68",
  "term_id": "GO:0007286"
}